{
  "gene_name": "U7 snRNA-associated Sm-like protein LSm11",
  "term_id": "GO:0006398",
  "term_label": "mRNA 3'-end processing by stem-loop binding and cleavage",
  "gene": "UniProtKB:P83369",
  "gene_symbol": "LSM11"
}